{
  "gene_name": "Short transient receptor potential channel 7",
  "gene_symbol": "TRPC7",
  "term_label": "inositol 1,4,5 trisphosphate binding",
  "gene": "UniProtKB:Q9HCX4",
  "term_id": "GO:0070679"
}